{
  "gene_name": "Divergent paired-related homeobox",
  "term_id": "GO:0006357",
  "gene_symbol": "DPRX",
  "gene": "UniProtKB:A6NFQ7",
  "term_label": "regulation of transcription by RNA polymerase II"
}